{
  "gene": "UniProtKB:P50539",
  "gene_name": "Max-interacting protein 1",
  "term_id": "GO:0006357",
  "gene_symbol": "MXI1",
  "term_label": "regulation of transcription by RNA polymerase II"
}